toll-like receptor 8 signaling pathway [GO:0034158] (biological process) Regulation: regulated by regulation of toll-like receptor 8 signaling pathway [GO:0034159]; negatively regulated by GO:0034160; positively regulated by GO:0034161 Definition: The series of molecular signals initiated by a ligand binding to the endolysosomal toll-like receptor 8. Also known as: TLR8 signaling pathway, toll-like receptor 8 signalling pathway References: PMID:16551253, PMID:17328678 Sources: GOC:add Relationships: is a type of endolysosomal toll-like receptor signaling pathway [GO:0140894]